{
  "term_label": "telomeric DNA binding",
  "gene_symbol": "SMG5",
  "gene_name": "Nonsense-mediated mRNA decay factor SMG5",
  "term_id": "GO:0042162",
  "gene": "UniProtKB:Q9UPR3"
}